{
  "term_id": "GO:0007346",
  "gene": "UniProtKB:Q8NHZ8",
  "term_label": "regulation of mitotic cell cycle",
  "gene_name": "Anaphase-promoting complex subunit CDC26",
  "gene_symbol": "CDC26"
}